{
  "gene_name": "C-type lectin domain family 17, member A",
  "term_label": "D-mannose binding",
  "gene": "UniProtKB:Q6ZS10",
  "term_id": "GO:0005537",
  "gene_symbol": "CLEC17A"
}